{
  "gene_name": "Retinol-binding protein 5",
  "term_id": "GO:0015908",
  "term_label": "fatty acid transport",
  "gene_symbol": "RBP5",
  "gene": "UniProtKB:P82980"
}